{
  "gene": "UniProtKB:Q8NBI5",
  "term_id": "UNKNOWN:0002",
  "gene_name": "Equilibrative nucleobase transporter 1",
  "term_label": "Unknown biological process",
  "gene_symbol": "SLC43A3"
}